{
  "term_label": "microtubule cytoskeleton organization",
  "gene": "UniProtKB:Q9Y4F4",
  "gene_symbol": "TOGARAM1",
  "term_id": "GO:0000226",
  "gene_name": "TOG array regulator of axonemal microtubules protein 1"
}